{
  "gene_name": "Protein ABHD1",
  "term_id": "GO:0051793",
  "gene_symbol": "ABHD1",
  "term_label": "medium-chain fatty acid catabolic process",
  "gene": "UniProtKB:Q96SE0"
}